{
  "gene_name": "Renin",
  "gene_symbol": "REN",
  "term_id": "GO:0002003",
  "term_label": "angiotensin maturation",
  "gene": "UniProtKB:P00797"
}